{
  "gene_name": "Beclin-1",
  "term_label": "phosphatidylinositol 3-kinase complex, class III, type II",
  "gene": "UniProtKB:Q14457",
  "term_id": "GO:0034272",
  "gene_symbol": "BECN1"
}